intracellular vesicle [GO:0097708] (cellular component) Relationships: is a type of vesicle [GO:0031982]; is a type of intracellular membrane-bounded organelle [GO:0043231] Sources: GOC:vesicles Subtypes: cytoplasmic vesicle [GO:0031410], virion transport vesicle [GO:0046816] Definition: Any vesicle that is part of the intracellular region.